{
  "gene_name": "Proline-rich protein 22",
  "term_label": "Unknown molecular function",
  "gene_symbol": "PRR22",
  "term_id": "UNKNOWN:0001",
  "gene": "UniProtKB:Q8IZ63"
}